{
  "gene_name": "MAP3K7 C-terminal-like protein",
  "term_id": "UNKNOWN:0002",
  "gene": "UniProtKB:P57077",
  "gene_symbol": "MAP3K7CL",
  "term_label": "Unknown biological process"
}